{
  "gene_symbol": "METTL15",
  "gene": "UniProtKB:A6NJ78",
  "gene_name": "12S rRNA N4-methylcytidine (m4C) methyltransferase",
  "term_label": "rRNA base methylation",
  "term_id": "GO:0070475"
}